{
  "gene": "UniProtKB:Q8IZF2",
  "gene_name": "Adhesion G protein-coupled receptor F5",
  "term_id": "GO:0004930",
  "gene_symbol": "ADGRF5",
  "term_label": "G protein-coupled receptor activity"
}